{
  "gene_name": "Small EDRK-rich factor 2",
  "gene_symbol": "SERF2",
  "gene": "UniProtKB:P84101",
  "term_id": "UNKNOWN:0003",
  "term_label": "Unknown cellular component"
}